{
  "term_label": "GPI anchor biosynthetic process",
  "term_id": "GO:0006506",
  "gene_name": "GPI inositol-deacylase",
  "gene": "UniProtKB:Q75T13",
  "gene_symbol": "PGAP1"
}